{
  "gene": "UniProtKB:P06756",
  "term_label": "integrin alphav-beta1 complex",
  "gene_symbol": "ITGAV",
  "term_id": "GO:0034682",
  "gene_name": "Integrin alpha-V"
}